{
  "term_label": "translation initiation factor binding",
  "gene_name": "Zinc finger protein ZPR1",
  "term_id": "GO:0031369",
  "gene_symbol": "ZPR1",
  "gene": "UniProtKB:O75312"
}